{
  "term_label": "Unknown biological process",
  "gene": "UniProtKB:Q8NEM8",
  "gene_symbol": "AGBL3",
  "term_id": "UNKNOWN:0002",
  "gene_name": "Cytosolic carboxypeptidase 3"
}